{
  "gene_symbol": "JAK3",
  "term_id": "GO:0042981",
  "gene": "UniProtKB:P52333",
  "term_label": "regulation of apoptotic process",
  "gene_name": "Tyrosine-protein kinase JAK3"
}